reproductive blastospore formation [GO:0034299] (biological process) Relationships: is a type of conidium formation [GO:0048315]; is a type of anatomical structure formation involved in morphogenesis [GO:0048646] Note: Note that this term should not be confused with the usage of 'blastospore' to mean any yeast-form fungal cell, as in Candida species. Definition: The formation of a spore following the marked enlargement of part of a cell before separation by a septum. Blastospores are a type of asexual spore found in some fungi, most notably the class Glomeromycota. References: PMID:30910084 Sources: GOC:mah Also known as: blastoconidium formation